{
  "gene_symbol": "SLC16A2",
  "term_id": "GO:0005886",
  "gene_name": "Monocarboxylate transporter 8",
  "gene": "UniProtKB:P36021",
  "term_label": "plasma membrane"
}